2-methylbutanoyl-CoA(4-) biosynthetic process [GO:1902191] (biological process) Also known as: 2-methylbutanoyl-CoA(4-) anabolism, 2-methylbutanoyl-CoA(4-) biosynthesis, 2-methylbutanoyl-CoA(4-) formation, 2-methylbutanoyl-CoA(4-) synthesis Definition: The chemical reactions and pathways resulting in the formation of 2-methylbutanoyl-CoA(4-). Relationships: is a type of fatty-acyl-CoA biosynthetic process [GO:0046949] References: PMID:15574432 Sources: GOC:TermGenie